{
  "gene_name": "Meiotic recombination protein REC8 homolog",
  "gene": "UniProtKB:O95072",
  "gene_symbol": "REC8",
  "term_label": "meiotic cohesin complex",
  "term_id": "GO:0030893"
}